{
  "gene_name": "Tripartite motif-containing protein 59",
  "gene_symbol": "TRIM59",
  "term_id": "GO:0045087",
  "gene": "UniProtKB:Q8IWR1",
  "term_label": "innate immune response"
}